{
  "gene_name": "Voltage-dependent L-type calcium channel subunit alpha-1F",
  "gene_symbol": "CACNA1F",
  "term_id": "GO:0008331",
  "gene": "UniProtKB:O60840",
  "term_label": "high voltage-gated calcium channel activity"
}